positive regulation of type 2 mitophagy [GO:1905091] (biological process) Definition: Any process that activates or increases the frequency, rate or extent of type 2 mitophagy. References: PMID:25009776, PMID:26942284 Sources: GOC:vw Relationships: is a type of positive regulation of mitophagy [GO:1901526]; is a type of regulation of type 2 mitophagy [GO:1905089]; positively regulates type 2 mitophagy [GO:0061734] Also known as: positive regulation of PRKN-mediated stimulation of mitophagy in response to mitochondrial depolarization, positive regulation of Park2-mediated stimulation of mitophagy in response to mitochondrial depolarization, positive regulation of parkin-mediated stimulation of mitophagy in response to mitochondrial depolarization, activation of parkin-mediated mitophagy in response to mitochondrial depolarization